{
  "term_label": "phospholipid transporter activity",
  "gene": "UniProtKB:P11597",
  "term_id": "GO:0005548",
  "gene_name": "Cholesteryl ester transfer protein",
  "gene_symbol": "CETP"
}